lung lobe development [GO:0060462] (biological process) Relationships: is a type of anatomical structure development [GO:0048856]; is part of lung development [GO:0030324] Definition: The biological process whose specific outcome is the progression of a lung lobe from an initial condition to its mature state. This process begins with the formation of a lung lobe by branching morphogenesis and ends with the mature structure. A lung lobe is one of the rounded projections that compose the lung. Sources: GOC:dph